meiotic spindle [GO:0072687] (cellular component) Relationships: is_a spindle [GO:0005819] References: PMID:11408572, PMID:18367542, PMID:8027178 Sources: GOC:mah, GOC:vw Definition: A spindle that forms as part of meiosis. Several proteins, such as budding yeast Spo21p, fission yeast Spo2 and Spo13, and C. elegans mei-1, localize specifically to the meiotic spindle and are absent from the mitotic spindle.